{
  "term_label": "plasma membrane",
  "gene_symbol": "CDH16",
  "term_id": "GO:0005886",
  "gene_name": "Cadherin-16",
  "gene": "UniProtKB:O75309"
}